symbiont-mediated activation of host transcription [GO:1990216] (biological process) Relationships: is a type of symbiont-mediated perturbation of host transcription [GO:0052026] Also known as: positive regulation by symbiont of host transcription References: PMID:21994350 Definition: A process in which a symbiont initiates, promotes, or enhances transcription of genes into mRNA in its host. The host is defined as the larger of the organisms involved in a symbiotic interaction.